{
  "gene_symbol": "ACKR2",
  "term_label": "calcium-mediated signaling",
  "term_id": "GO:0019722",
  "gene": "UniProtKB:O00590",
  "gene_name": "Atypical chemokine receptor 2"
}